{
  "term_label": "structural constituent of cytoskeleton",
  "term_id": "GO:0005200",
  "gene_symbol": "TUBA3C",
  "gene": "UniProtKB:P0DPH7",
  "gene_name": "Tubulin alpha-3C chain"
}